{
  "term_id": "GO:0031430",
  "term_label": "M band",
  "gene": "UniProtKB:Q14324",
  "gene_name": "Myosin-binding protein C, fast-type",
  "gene_symbol": "MYBPC2"
}